metanephric nephron development [GO:0072210] (biological process) Relationships: is a type of nephron development [GO:0072006]; BFO_0000050 metanephros development [GO:0001656] Definition: The process whose specific outcome is the progression of a nephron in the metanephros over time, from its formation to the mature structure. A nephron is the functional unit of the kidney. Subtypes: metanephric long nephron development [GO:0072238], metanephric short nephron development [GO:0072270] Sources: GOC:mtg_kidney_jan10